{
  "gene_name": "Kelch-like protein 11",
  "term_label": "proteasome-mediated ubiquitin-dependent protein catabolic process",
  "gene": "UniProtKB:Q9NVR0",
  "gene_symbol": "KLHL11",
  "term_id": "GO:0043161"
}